{
  "gene_symbol": "LAIR2",
  "gene_name": "Leukocyte-associated immunoglobulin-like receptor 2",
  "term_label": "plasma membrane",
  "gene": "UniProtKB:Q6ISS4",
  "term_id": "GO:0005886"
}